{
  "gene_symbol": "CD300A",
  "term_id": "GO:0004888",
  "term_label": "transmembrane signaling receptor activity",
  "gene_name": "CMRF35-like molecule 8",
  "gene": "UniProtKB:Q9UGN4"
}